{
  "gene_name": "Signal-induced proliferation-associated 1-like protein 1",
  "gene_symbol": "SIPA1L1",
  "gene": "UniProtKB:O43166",
  "term_label": "GTPase activator activity",
  "term_id": "GO:0005096"
}